{
  "term_id": "GO:0050727",
  "gene": "UniProtKB:P59044",
  "gene_symbol": "NLRP6",
  "term_label": "regulation of inflammatory response",
  "gene_name": "NACHT, LRR and PYD domains-containing protein 6"
}